{
  "gene": "UniProtKB:O00148",
  "gene_name": "ATP-dependent RNA helicase DDX39A",
  "term_label": "Unknown cellular component",
  "term_id": "UNKNOWN:0003",
  "gene_symbol": "DDX39A"
}